{
  "gene_name": "ADP-ribosylation factor 1",
  "term_id": "GO:0005886",
  "gene_symbol": "ARF1",
  "term_label": "plasma membrane",
  "gene": "UniProtKB:P84077"
}